regulation of vacuole fusion, non-autophagic [GO:0032889] (biological process) Relationships: is_a regulation of vacuole organization [GO:0044088]; regulates vacuole fusion, non-autophagic [GO:0042144] Subtypes: positive regulation of vacuole fusion, non-autophagic [GO:0061191], negative regulation of vacuole fusion, non-autophagic [GO:0061192] Sources: GOC:mah Definition: Any process that modulates the frequency, rate or extent of the fusion of two vacuole membranes to form a single vacuole.